{
  "gene_name": "Sphingosine-1-phosphate transporter SPNS2",
  "gene_symbol": "SPNS2",
  "gene": "UniProtKB:Q8IVW8",
  "term_id": "GO:0022857",
  "term_label": "transmembrane transporter activity"
}